negative regulation of translation in response to stress [GO:0032055] (biological process) Also known as: down regulation of translation in response to stress, down-regulation of translation in response to stress, downregulation of translation in response to stress, inhibition of translation in response to stress Subtypes: negative regulation of translation in response to osmotic stress [GO:0032061], regulation of translation in response to oxidative stress [GO:0043556], negative regulation of translational initiation in response to starvation [GO:0071263], sucrose induced translational repression [GO:0080149], GO:1902010, negative regulation of cytoplasmic translational initiation in response to stress [GO:1990625] Sources: GOC:mah Definition: Any process that stops, prevents or reduces the rate of translation as a result of a stimulus indicating the organism is under stress. Relationships: is a type of negative regulation of translation [GO:0017148]; is a type of GO:0043555